{
  "term_id": "GO:0006508",
  "gene_symbol": "ADAMTS5",
  "term_label": "proteolysis",
  "gene": "UniProtKB:Q9UNA0",
  "gene_name": "A disintegrin and metalloproteinase with thrombospondin motifs 5"
}